positive regulation of atrial cardiac muscle cell action potential [GO:1903949] (biological process) Also known as: up regulation of atrial cardiac muscle cell action potential, up-regulation of atrial cardiac muscle cell action potential, upregulation of atrial cardiac muscle cell action potential, activation of atrial cardiac muscle cell action potential References: PMID:25281747 Sources: GOC:BHF, GOC:TermGenie, GOC:mtg_cardiac_conduct_nov11, GOC:nc, GO_REF:0000058 Relationships: is a type of GO:0045760; is a type of regulation of atrial cardiac muscle cell action potential [GO:0098910]; positively regulates GO:0086014 Definition: Any process that activates or increases the frequency, rate or extent of atrial cardiac muscle cell action potential.